{
  "term_label": "L-glutamate transmembrane transporter activity",
  "gene": "UniProtKB:P43005",
  "term_id": "GO:0005313",
  "gene_symbol": "SLC1A1",
  "gene_name": "Excitatory amino acid transporter 3"
}